mitochondrion-plasma membrane adaptor activity [GO:0140443] (molecular function) Also known as: mitochondrion plasma membrane adaptor activity, mitochondrion plasma membrane tether activity, plasma membrane-mitochondrion adaptor activity, plasma membrane-mitochondrion tether activity Relationships: is a type of protein-membrane adaptor activity [GO:0043495] References: PMID:31582398 Definition: The binding activity of a molecule that brings together a mitochondrion and a plasma membrane either via membrane lipid binding or by interacting with a mitochondrial outer membrane protein, to establish or maintain the localization of the mitochondrion.